{
  "gene": "UniProtKB:O95396",
  "term_id": "GO:0042292",
  "gene_name": "Adenylyltransferase and sulfurtransferase MOCS3",
  "term_label": "URM1 activating enzyme activity",
  "gene_symbol": "MOCS3"
}